{
  "term_label": "plasma membrane",
  "term_id": "GO:0005886",
  "gene_symbol": "NPY1R",
  "gene_name": "Neuropeptide Y receptor type 1",
  "gene": "UniProtKB:P25929"
}